{
  "gene": "UniProtKB:P52895",
  "term_id": "GO:0044597",
  "gene_symbol": "AKR1C2",
  "gene_name": "Aldo-keto reductase family 1 member C2",
  "term_label": "daunorubicin metabolic process"
}